{
  "gene_name": "Procollagen C-endopeptidase enhancer 1",
  "gene": "UniProtKB:Q15113",
  "term_id": "GO:0005518",
  "gene_symbol": "PCOLCE",
  "term_label": "collagen binding"
}